{
  "gene": "UniProtKB:Q494W8",
  "gene_symbol": "CHRFAM7A",
  "gene_name": "CHRNA7-FAM7A fusion protein",
  "term_label": "acetylcholine-gated channel complex",
  "term_id": "GO:0005892"
}